{
  "gene": "UniProtKB:Q969Q1",
  "term_id": "GO:0005737",
  "term_label": "cytoplasm",
  "gene_name": "E3 ubiquitin-protein ligase TRIM63",
  "gene_symbol": "TRIM63"
}